{
  "term_id": "GO:0004867",
  "gene_name": "Serpin B3",
  "gene_symbol": "SERPINB3",
  "gene": "UniProtKB:P29508",
  "term_label": "serine-type endopeptidase inhibitor activity"
}